{
  "term_label": "Unknown biological process",
  "gene_name": "Pre-mRNA-splicing factor SYF2",
  "term_id": "UNKNOWN:0002",
  "gene_symbol": "SYF2",
  "gene": "UniProtKB:O95926"
}